{
  "gene_name": "Adenosine 3'-phospho 5'-phosphosulfate transporter 2",
  "term_id": "GO:0055085",
  "term_label": "transmembrane transport",
  "gene_symbol": "SLC35B3",
  "gene": "UniProtKB:Q9H1N7"
}